regulation of blood pressure by chemoreceptor signaling pathway [GO:0010850] (biological process) Sources: GOC:dph, GOC:tb Relationships: is a type of signal transduction [GO:0007165]; is a type of regulation of blood pressure [GO:0008217] Definition: A series of reactions within the cell that occur as a result of a single trigger reaction or compound interacting with a chemoreceptor resulting in a modulation of the force with which blood travels through the circulatory system. Chemoreceptors respond to oxygen, carbon dioxide and hydrogen ions. Also known as: regulation of blood pressure by chemoreceptor signalling pathway